{
  "gene_symbol": "HEATR5A",
  "gene_name": "HEAT repeat-containing protein 5A",
  "gene": "UniProtKB:Q86XA9",
  "term_label": "Unknown molecular function",
  "term_id": "UNKNOWN:0001"
}